1-(4-iodo-2,5-dimethoxyphenyl)propan-2-amine binding [GO:0071886] (molecular function) Definition: Binding to the amine 1-(4-iodo-2,5-dimethoxyphenyl)propan-2-amine, a serotonin receptor agonist that can act as a psychedelic drug. References: PMID:19057895 Sources: GOC:yaf Also known as: (+/-)2-(4-iodo-2,5-dimethoxy-phenyl)-1-methyl-ethylamine binding, 1-(4-iodo-2,5-dimethoxyphenyl)-2-aminopropane binding, 4-iodo-2,5-dimethoxyphenylisopropylamine binding Relationships: is a type of amine binding [GO:0043176]